{
  "gene": "UniProtKB:A8MX34",
  "gene_symbol": "KRTAP29-1",
  "term_label": "Unknown biological process",
  "gene_name": "Keratin-associated protein 29-1",
  "term_id": "UNKNOWN:0002"
}